{
  "term_id": "GO:0001664",
  "gene_name": "Beta-arrestin-1",
  "gene": "UniProtKB:P49407",
  "gene_symbol": "ARRB1",
  "term_label": "G protein-coupled receptor binding"
}